{
  "term_id": "GO:0000045",
  "gene_name": "Autophagy protein 5",
  "gene": "UniProtKB:Q9H1Y0",
  "term_label": "autophagosome assembly",
  "gene_symbol": "ATG5"
}